{
  "gene_symbol": "PCDHA5",
  "gene": "UniProtKB:Q9Y5H7",
  "gene_name": "Protocadherin alpha-5",
  "term_label": "plasma membrane",
  "term_id": "GO:0005886"
}